mitochondrial intermembrane space chaperone complex [GO:0042719] (cellular component) Also known as: small TIM complex, Tim8-Tim13 complex, Tim9-Tim10 complex, mitochondrial intermembrane space protein transporter complex Sources: GOC:vw Relationships: is a type of mitochondrial protein-containing complex [GO:0098798]; is part of mitochondrial intermembrane space [GO:0005758] Definition: mitochondrial protein-containing complex localised in the mitochondrial inner membrane space that chaperones proteins to the TIM22 complex for insertion into the mitochondrial inner membrane.